{
  "term_id": "UNKNOWN:0001",
  "gene_name": "Leptin receptor overlapping transcript-like 1",
  "gene_symbol": "LEPROTL1",
  "term_label": "Unknown molecular function",
  "gene": "UniProtKB:O95214"
}